alpha-copaene synthase activity [GO:0102877] (molecular function) Definition: Catalysis of the reaction: 2-trans,6-trans-farnesyl diphosphate = alpha-copaene + diphosphoric acid. Sources: EC:4.2.3.133, GOC:pz Relationships: is_a GO:0016838